T cell chemotaxis [GO:0010818] (biological process) Definition: The directed movement of a T cell in response to an external stimulus. A T cell is a type of lymphocyte whose defining characteristic is the expression of a T cell receptor complex. Sources: GOC:dph, GOC:tb Also known as: T-cell chemotaxis Relationships: is a type of GO:0048247; is a type of GO:0072678 Subtypes: helper T cell chemotaxis [GO:0035704], T-helper 17 cell chemotaxis [GO:0035705], GO:0035706, T-helper 2 cell chemotaxis [GO:0035707] Regulation: regulated by GO:0010819; positively regulated by positive regulation of T cell chemotaxis [GO:0010820]